{
  "gene": "UniProtKB:P55209",
  "term_label": "chromatin",
  "gene_name": "Nucleosome assembly protein 1-like 1",
  "term_id": "GO:0000785",
  "gene_symbol": "NAP1L1"
}